{
  "gene_symbol": "IL18RAP",
  "term_id": "GO:0035655",
  "gene_name": "Interleukin-18 receptor accessory protein",
  "term_label": "interleukin-18-mediated signaling pathway",
  "gene": "UniProtKB:O95256"
}